{
  "gene": "UniProtKB:O43493",
  "term_id": "UNKNOWN:0002",
  "term_label": "Unknown biological process",
  "gene_symbol": "TGOLN2",
  "gene_name": "Trans-Golgi network integral membrane protein 2"
}